{
  "gene_name": "Uncharacterized protein C2orf27A",
  "gene": "UniProtKB:P0DPF5",
  "term_label": "Unknown cellular component",
  "gene_symbol": "C2orf27A",
  "term_id": "UNKNOWN:0003"
}